{
  "gene_symbol": "Q9N2K0",
  "term_label": "Unknown molecular function",
  "gene_name": "HERV-H_2q24.3 provirus ancestral Env polyprotein",
  "gene": "UniProtKB:Q9N2K0",
  "term_id": "UNKNOWN:0001"
}